{
  "term_label": "Unknown molecular function",
  "gene": "UniProtKB:Q9Y625",
  "gene_name": "Glypican-6",
  "gene_symbol": "GPC6",
  "term_id": "UNKNOWN:0001"
}